{
  "gene_name": "Uncharacterized protein C16orf78",
  "term_id": "UNKNOWN:0003",
  "gene_symbol": "C16orf78",
  "term_label": "Unknown cellular component",
  "gene": "UniProtKB:Q8WTQ4"
}